{
  "gene_name": "Testis-specific H1 histone",
  "gene_symbol": "H1-7",
  "term_id": "GO:0005634",
  "term_label": "nucleus",
  "gene": "UniProtKB:Q75WM6"
}